{
  "term_id": "UNKNOWN:0002",
  "term_label": "Unknown biological process",
  "gene_name": "Regulator of microtubule dynamics protein 1",
  "gene_symbol": "RMDN1",
  "gene": "UniProtKB:Q96DB5"
}